{
  "term_label": "cytoplasm",
  "gene_symbol": "EIF4ENIF1",
  "gene": "UniProtKB:Q9NRA8",
  "term_id": "GO:0005737",
  "gene_name": "Eukaryotic translation initiation factor 4E transporter"
}